{
  "gene_name": "Uncharacterized protein DNAH10OS",
  "gene": "UniProtKB:P0CZ25",
  "gene_symbol": "DNAH10OS",
  "term_id": "UNKNOWN:0001",
  "term_label": "Unknown molecular function"
}